NAD-malic enzyme C4 photosynthesis [GO:0009763] (biological process) Definition: The process of C4 photosynthesis, as it occurs in plants in which the enzyme decarboxylating C4 acids in the bundle sheath is NAD-malic enzyme. References: PMID:11788762 Relationships: is_a C4 photosynthesis [GO:0009760]